male germ-line stem cell asymmetric division [GO:0048133] (BP) Definition: The self-renewing division of a germline stem cell in the male gonad, to produce a daughter stem cell and a daughter germ cell, which will divide to form the male gametes. Sources: GOC:jid Also known as: male germ-line stem cell renewal Relationships: is a type of germline stem cell asymmetric division [GO:0098728]; is part of GO:0007283 Regulation: regulated by regulation of male germ-line stem cell asymmetric division [GO:1904838]; negatively regulated by negative regulation of male germ-line stem cell asymmetric division [GO:1904839]; positively regulated by positive regulation of male germ-line stem cell asymmetric division [GO:1904840]